{
  "term_id": "GO:0045109",
  "gene_symbol": "KRT77",
  "gene": "UniProtKB:Q7Z794",
  "term_label": "intermediate filament organization",
  "gene_name": "Keratin, type II cytoskeletal 1b"
}